{
  "gene_symbol": "KIF25-AS1",
  "gene_name": "Putative uncharacterized protein KIF25-AS1",
  "term_label": "Unknown cellular component",
  "term_id": "UNKNOWN:0003",
  "gene": "UniProtKB:Q9Y6Z4"
}